{
  "term_label": "Unknown biological process",
  "gene_name": "Immunoglobulin-like and fibronectin type III domain-containing protein 1",
  "term_id": "UNKNOWN:0002",
  "gene_symbol": "IGFN1",
  "gene": "UniProtKB:Q86VF2"
}